{
  "gene": "UniProtKB:Q9NQW8",
  "gene_symbol": "CNGB3",
  "gene_name": "Cyclic nucleotide-gated cation channel beta-3",
  "term_label": "plasma membrane",
  "term_id": "GO:0005886"
}